{
  "gene_symbol": "KANSL3",
  "term_id": "UNKNOWN:0001",
  "term_label": "Unknown molecular function",
  "gene": "UniProtKB:Q9P2N6",
  "gene_name": "KAT8 regulatory NSL complex subunit 3"
}